{
  "term_id": "GO:0019957",
  "term_label": "C-C chemokine binding",
  "gene_symbol": "CXCR1",
  "gene_name": "C-X-C chemokine receptor type 1",
  "gene": "UniProtKB:P25024"
}